response to metal ion [GO:0010038] (biological process) Sources: GOC:sm Definition: Any process that results in a change in state or activity of a cell or an organism (in terms of movement, secretion, enzyme production, gene expression, etc.) as a result of a metal ion stimulus. Also known as: response to metal, response to heavy metal, heavy metal sensitivity/resistance Subtypes: response to iron ion [GO:0010039], response to manganese ion [GO:0010042], response to zinc ion [GO:0010043], response to aluminum ion [GO:0010044], response to nickel cation [GO:0010045], response to cesium ion [GO:0010164], GO:0010226, response to silver ion [GO:0010272], response to lead ion [GO:0010288], GO:0032025, GO:0032026, response to potassium ion [GO:0035864], response to cadmium ion [GO:0046686], response to copper ion [GO:0046688], response to mercury ion [GO:0046689], response to calcium ion [GO:0051592], response to platinum ion [GO:0070541], cellular response to metal ion [GO:0071248], stress response to metal ion [GO:0097501], GO:1904311 Relationships: is a type of response to chemical [GO:0042221]